{
  "gene": "UniProtKB:Q9UPY8",
  "term_label": "protein localization to microtubule",
  "gene_name": "Microtubule-associated protein RP_EB family member 3",
  "term_id": "GO:0035372",
  "gene_symbol": "MAPRE3"
}